{
  "gene_name": "Acylphosphatase-2",
  "gene_symbol": "ACYP2",
  "term_id": "UNKNOWN:0003",
  "term_label": "Unknown cellular component",
  "gene": "UniProtKB:P14621"
}